{
  "term_id": "UNKNOWN:0002",
  "gene_symbol": "CMAS",
  "gene": "UniProtKB:Q8NFW8",
  "gene_name": "N-acylneuraminate cytidylyltransferase",
  "term_label": "Unknown biological process"
}